{
  "term_label": "Unknown biological process",
  "gene": "UniProtKB:Q3ZCQ3",
  "gene_symbol": "FAM174B",
  "gene_name": "Membrane protein FAM174B",
  "term_id": "UNKNOWN:0002"
}